oxidative RNA demethylase activity [GO:0035515] (molecular function) Subtypes: GO:1990930, mRNA N6-methyladenosine dioxygenase activity [GO:1990931], tRNA demethylase activity [GO:1990984] Definition: Catalysis of the removal of a methyl group from one or more nucleosides within a RNA molecule involving the oxidation (i.e. electron loss) of one or more atoms. Relationships: is a type of 2-oxoglutarate-dependent dioxygenase activity [GO:0016706]; is a type of demethylase activity [GO:0032451]; is a type of catalytic activity, acting on RNA [GO:0140098] References: PMID:12594517, PMID:16482161, PMID:18775698 Also known as: 2-oxoglutarate-dependent RNA demethylase